{
  "term_label": "Unknown biological process",
  "gene": "UniProtKB:Q6UWV6",
  "term_id": "UNKNOWN:0002",
  "gene_name": "Ectonucleotide pyrophosphatase_phosphodiesterase family member 7",
  "gene_symbol": "ENPP7"
}